{
  "term_label": "gonadotropin-releasing hormone receptor activity",
  "gene_symbol": "GPR173",
  "gene_name": "Probable G-protein coupled receptor 173",
  "gene": "UniProtKB:Q9NS66",
  "term_id": "GO:0004968"
}